{
  "gene": "UniProtKB:Q16643",
  "term_id": "UNKNOWN:0002",
  "gene_symbol": "DBN1",
  "gene_name": "Drebrin",
  "term_label": "Unknown biological process"
}